{
  "gene_name": "Protein ripply1",
  "term_label": "negative regulation of transcription by RNA polymerase II",
  "term_id": "GO:0000122",
  "gene": "UniProtKB:Q0D2K3",
  "gene_symbol": "RIPPLY1"
}